{
  "gene_symbol": "WNT5A",
  "gene_name": "Protein Wnt-5a",
  "term_label": "neuron differentiation",
  "gene": "UniProtKB:P41221",
  "term_id": "GO:0030182"
}